oocyte animal/vegetal axis specification [GO:0060832] (BP) Relationships: is a type of oocyte axis specification [GO:0007309] Sources: GOC:dph, GOC:sdb_2009, GOC:tb Definition: The establishment, maintenance and elaboration of the animal/vegetal axis in the oocyte. The animal/vegetal axis of an oocyte is defined by the placement of the nucleus in the oocyte and can sometimes be identified by the asymmetric placement of other substances such as yolk in the oocyte. The pole of the egg that is closest to the nucleus defines the animal end, with the axis passing through the nucleus.